{
  "gene_symbol": "MLLT3",
  "gene_name": "Protein AF-9",
  "gene": "UniProtKB:P42568",
  "term_label": "chromatin binding",
  "term_id": "GO:0003682"
}